{
  "gene_name": "G1_S-specific cyclin-E1",
  "term_id": "GO:0016538",
  "gene_symbol": "CCNE1",
  "gene": "UniProtKB:P24864",
  "term_label": "cyclin-dependent protein serine/threonine kinase regulator activity"
}